{
  "gene_symbol": "CRNKL1",
  "gene": "UniProtKB:Q9BZJ0",
  "gene_name": "Crooked neck-like protein 1",
  "term_id": "GO:0071014",
  "term_label": "post-mRNA release spliceosomal complex"
}